{
  "gene_name": "Interleukin-36 alpha",
  "term_label": "cytokine activity",
  "gene_symbol": "IL36A",
  "gene": "UniProtKB:Q9UHA7",
  "term_id": "GO:0005125"
}